{
  "term_id": "UNKNOWN:0002",
  "gene_name": "Leucine-rich repeat-containing protein 56",
  "gene": "UniProtKB:Q8IYG6",
  "gene_symbol": "LRRC56",
  "term_label": "Unknown biological process"
}